{
  "gene": "UniProtKB:P09683",
  "gene_name": "Secretin",
  "term_id": "GO:0007420",
  "gene_symbol": "SCT",
  "term_label": "brain development"
}